{
  "gene_symbol": "NCAM2",
  "gene": "UniProtKB:O15394",
  "term_label": "Unknown biological process",
  "gene_name": "Neural cell adhesion molecule 2",
  "term_id": "UNKNOWN:0002"
}